{
  "term_id": "GO:0030198",
  "term_label": "extracellular matrix organization",
  "gene_symbol": "ADAMTS18",
  "gene_name": "A disintegrin and metalloproteinase with thrombospondin motifs 18",
  "gene": "UniProtKB:Q8TE60"
}